{
  "gene": "UniProtKB:Q13561",
  "gene_symbol": "DCTN2",
  "term_label": "dynactin complex",
  "term_id": "GO:0005869",
  "gene_name": "Dynactin subunit 2"
}